{
  "term_label": "collagen fibril organization",
  "gene_symbol": "DPT",
  "term_id": "GO:0030199",
  "gene": "UniProtKB:Q07507",
  "gene_name": "Dermatopontin"
}